{
  "gene_name": "Astrocytic phosphoprotein PEA-15",
  "gene": "UniProtKB:Q15121",
  "term_label": "negative regulation of extrinsic apoptotic signaling pathway via death domain receptors",
  "gene_symbol": "PEA15",
  "term_id": "GO:1902042"
}